{
  "gene_symbol": "RALGAPB",
  "term_label": "Ral protein signal transduction",
  "term_id": "GO:0032484",
  "gene_name": "Ral GTPase-activating protein subunit beta",
  "gene": "UniProtKB:Q86X10"
}